{
  "gene_symbol": "TBC1D7",
  "gene_name": "TBC1 domain family member 7",
  "gene": "UniProtKB:Q9P0N9",
  "term_label": "negative regulation of TOR signaling",
  "term_id": "GO:0032007"
}